{
  "term_id": "UNKNOWN:0002",
  "gene": "UniProtKB:Q8N7B9",
  "term_label": "Unknown biological process",
  "gene_symbol": "EFCAB3",
  "gene_name": "EF-hand calcium-binding domain-containing protein 3"
}